{
  "gene_symbol": "FAM110A",
  "term_label": "Unknown molecular function",
  "term_id": "UNKNOWN:0001",
  "gene": "UniProtKB:Q9BQ89",
  "gene_name": "Protein FAM110A"
}